{
  "term_id": "UNKNOWN:0002",
  "gene_name": "Armadillo-like helical domain-containing protein 4",
  "term_label": "Unknown biological process",
  "gene_symbol": "ARMH4",
  "gene": "UniProtKB:Q86TY3"
}